{
  "term_label": "Unknown biological process",
  "term_id": "UNKNOWN:0002",
  "gene_name": "Putative uncharacterized protein LINC02693",
  "gene_symbol": "LINC02693",
  "gene": "UniProtKB:A8MQB3"
}